{
  "term_label": "glutamatergic synapse",
  "gene_symbol": "EFNB2",
  "gene": "UniProtKB:P52799",
  "term_id": "GO:0098978",
  "gene_name": "Ephrin-B2"
}